{
  "term_id": "UNKNOWN:0001",
  "gene_name": "WD repeat-containing protein WRAP73",
  "gene": "UniProtKB:Q9P2S5",
  "term_label": "Unknown molecular function",
  "gene_symbol": "WRAP73"
}